{
  "term_id": "GO:0005634",
  "term_label": "nucleus",
  "gene": "UniProtKB:Q92771",
  "gene_name": "Putative ATP-dependent RNA helicase DDX12",
  "gene_symbol": "DDX12P"
}